benzoyl-CoA biosynthetic process [GO:1901789] (biological process) Relationships: is a type of acyl-CoA biosynthetic process [GO:0071616]; is a type of benzoyl-CoA metabolic process [GO:1901787] Sources: GOC:TermGenie, GOC:yaf Definition: The chemical reactions and pathways resulting in the formation of benzoyl-CoA. Also known as: benzoyl-CoA anabolism, benzoyl-CoA biosynthesis, benzoyl-CoA formation, benzoyl-CoA synthesis